{
  "term_label": "Unknown biological process",
  "term_id": "UNKNOWN:0002",
  "gene": "UniProtKB:Q8WWI1",
  "gene_symbol": "LMO7",
  "gene_name": "LIM domain only protein 7"
}